trichome papilla formation [GO:1905499] (biological process) Relationships: is a type of GO:0010927; is a type of cell projection assembly [GO:0030031]; is part of trichome morphogenesis [GO:0010090] Also known as: trichome papilla assembly References: PMID:24014871 Sources: GOC:TermGenie, GOC:tb, GO_REF:0000079 Definition: The aggregation, arrangement and bonding together of a set of components to form a trichome papilla.